{
  "gene_name": "Fibroblast growth factor receptor 4",
  "gene_symbol": "FGFR4",
  "term_label": "positive regulation of cell population proliferation",
  "gene": "UniProtKB:P22455",
  "term_id": "GO:0008284"
}